{
  "term_id": "GO:0070291",
  "term_label": "N-acylethanolamine metabolic process",
  "gene": "UniProtKB:Q9NZC3",
  "gene_symbol": "GDE1",
  "gene_name": "Glycerophosphodiester phosphodiesterase 1"
}